{
  "term_id": "GO:0005179",
  "term_label": "hormone activity",
  "gene_name": "Endothelin-2",
  "gene_symbol": "EDN2",
  "gene": "UniProtKB:P20800"
}